positive regulation of fibronectin-dependent thymocyte migration [GO:2000415] (BP) Relationships: is a type of GO:2000412; is a type of GO:2000413; positively regulates fibronectin-dependent thymocyte migration [GO:0072681] Definition: Any process that activates or increases the frequency, rate or extent of fibronectin-dependent thymocyte migration. Sources: GOC:BHF, GOC:mah Also known as: positive regulation of fibronectin-dependent thymic lymphocyte migration, positive regulation of fibronectin-dependent immature T cell migration, positive regulation of fibronectin-dependent immature T lymphocyte migration, positive regulation of fibronectin-dependent immature T-cell migration, positive regulation of fibronectin-dependent immature T-lymphocyte migration